{
  "gene_symbol": "C1QA",
  "gene_name": "Complement C1q subcomponent subunit A",
  "term_id": "UNKNOWN:0001",
  "gene": "UniProtKB:P02745",
  "term_label": "Unknown molecular function"
}